negative regulation of smooth muscle hypertrophy [GO:1905148] (biological process) Definition: Any process that stops, prevents or reduces the frequency, rate or extent of smooth muscle hypertrophy. References: PMID:22161164 Sources: GOC:BHF, GOC:BHF_miRNA, GOC:TermGenie, GOC:bc, GO_REF:0000058 Also known as: down regulation of smooth muscle hypertrophy, down-regulation of smooth muscle hypertrophy, downregulation of smooth muscle hypertrophy, inhibition of smooth muscle hypertrophy Relationships: is a type of GO:0014741; is a type of negative regulation of muscle adaptation [GO:0014745]; is a type of regulation of smooth muscle hypertrophy [GO:1905147]; negatively regulates smooth muscle hypertrophy [GO:0014895]